{
  "gene": "UniProtKB:Q04206",
  "term_label": "nucleus",
  "term_id": "GO:0005634",
  "gene_symbol": "RELA",
  "gene_name": "Transcription factor p65"
}